{
  "term_label": "late endosome",
  "gene": "UniProtKB:Q9NUS5",
  "gene_name": "AP-5 complex subunit sigma-1",
  "gene_symbol": "AP5S1",
  "term_id": "GO:0005770"
}